{
  "term_label": "[pyruvate dehydrogenase (acetyl-transferring)]-phosphatase activity",
  "gene": "UniProtKB:Q9P2J9",
  "gene_symbol": "PDP2",
  "gene_name": "[Pyruvate dehydrogenase [acetyl-transferring]]-phosphatase 2, mitochondrial",
  "term_id": "GO:0004741"
}